{
  "gene_symbol": "DAOA",
  "term_id": "UNKNOWN:0002",
  "term_label": "Unknown biological process",
  "gene_name": "D-amino acid oxidase activator",
  "gene": "UniProtKB:P59103"
}